{
  "term_id": "GO:0003735",
  "gene_name": "Small ribosomal subunit protein uS19",
  "gene": "UniProtKB:P62841",
  "term_label": "structural constituent of ribosome",
  "gene_symbol": "RPS15"
}